{
  "gene_symbol": "CYP2E1",
  "term_label": "arachidonate epoxygenase activity",
  "gene": "UniProtKB:P05181",
  "term_id": "GO:0008392",
  "gene_name": "Cytochrome P450 2E1"
}